positive regulation of urine volume [GO:0035810] (biological process) Sources: GOC:mtg_25march11, GOC:yaf Also known as: diuresis, elevation of urinary volume, increase in urine flow Definition: Any process that increases the amount of urine excreted from the body over a unit of time. Subtypes: positive regulation of urine volume by pressure natriuresis [GO:0035818] Relationships: is_a regulation of urine volume [GO:0035809]